positive regulation of killing of cells of another organism [GO:0051712] (biological process) Relationships: is a type of positive regulation of cell killing [GO:0031343]; is a type of positive regulation of programmed cell death [GO:0043068]; is a type of regulation of killing of cells of another organism [GO:0051709]; positively regulates killing of cells of another organism [GO:0031640] Also known as: positive regulation of killing of cells of other organism, up regulation of killing of cells of another organism, up-regulation of killing of cells of another organism, upregulation of killing of cells of another organism, activation of killing of cells of another organism, stimulation of killing of cells of another organism, activation by organism of apoptotic programmed cell death in other organism during symbiotic interaction, enhancement of other organism programmed cell death by organism Sources: GOC:ai Subtypes: positive regulation of neutrophil mediated killing of symbiont cell [GO:0070961] Definition: Any process that activates or increases the frequency, rate or extent of the killing by an organism of cells in another organism.